ecdysone O-acyltransferase activity [GO:0004173] (molecular function) Definition: Catalysis of the reaction: Ecdysone + palmitoyl-CoA = CoA + ecdysone palmitate. Sources: EC:2.3.1.139, RHEA:15217 Relationships: is a type of O-acyltransferase activity [GO:0008374] Also known as: acyl-CoA:ecdysone acyltransferase activity, fatty acyl-CoA:ecdysone acyltransferase activity, palmitoyl-CoA:ecdysone palmitoyltransferase activity